{
  "gene_name": "Cytoplasmic polyadenylation element-binding protein 3",
  "gene_symbol": "CPEB3",
  "gene": "UniProtKB:Q8NE35",
  "term_id": "GO:0005634",
  "term_label": "nucleus"
}